{
  "term_id": "GO:0072344",
  "gene_symbol": "NEMF",
  "gene": "UniProtKB:O60524",
  "gene_name": "Ribosome quality control complex subunit NEMF",
  "term_label": "rescue of stalled ribosome"
}